{
  "gene": "UniProtKB:Q96P66",
  "gene_symbol": "GPR101",
  "term_id": "GO:0005886",
  "term_label": "plasma membrane",
  "gene_name": "Probable G-protein coupled receptor 101"
}